elastic fiber [GO:0071953] (cellular component) Relationships: is a type of GO:0099512; is part of GO:0031012 Also known as: elastic fibre, elastin fiber Definition: An supramolecular fiber that consists of an insoluble core of polymerized tropoelastin monomers and a surrounding mantle of microfibrils. Elastic fibers provide elasticity and recoiling to tissues and organs, and maintain structural integrity against mechanical strain. References: PMID:20236620 Sources: GOC:BHF, GOC:mah